{
  "gene_name": "Nuclear factor of activated T-cells 5",
  "term_id": "GO:0033173",
  "term_label": "calcineurin-NFAT signaling cascade",
  "gene": "UniProtKB:O94916",
  "gene_symbol": "NFAT5"
}